{
  "gene": "UniProtKB:Q5T7P3",
  "gene_symbol": "LCE1B",
  "term_label": "Unknown molecular function",
  "gene_name": "Late cornified envelope protein 1B",
  "term_id": "UNKNOWN:0001"
}